morphogenesis of an epithelium [GO:0002009] (biological process) Definition: The process in which the anatomical structures of epithelia are generated and organized. An epithelium consists of closely packed cells arranged in one or more layers, that covers the outer surfaces of the body or lines any internal cavity or tube. Also known as: epithelium morphogenesis Subtypes: morphogenesis of a polarized epithelium [GO:0001738], morphogenesis of an epithelial sheet [GO:0002011], morphogenesis of an endothelium [GO:0003159], heart rudiment morphogenesis [GO:0003314], GO:0007441, GO:0016331, morphogenesis of follicular epithelium [GO:0016333], morphogenesis of larval imaginal disc epithelium [GO:0016335], initiation of neural tube closure [GO:0021993], epidermis morphogenesis [GO:0048730], GO:0060026, GO:0060562, morphogenesis of an epithelial fold [GO:0060571], GO:0060600, GO:0060601, GO:0060679, prostate gland epithelium morphogenesis [GO:0060740], clearance of cells from fusion plate [GO:0060884], morphogenesis of a branching epithelium [GO:0061138], renal vesicle morphogenesis [GO:0072077], nephron epithelium morphogenesis [GO:0072088], GO:0097536 Regulation: RO_0002211 by regulation of morphogenesis of an epithelium [GO:1905330]; negatively regulated by negative regulation of morphogenesis of an epithelium [GO:1905331]; positively regulated by positive regulation of morphogenesis of an epithelium [GO:1905332] Sources: GOC:dph, GOC:jl, GOC:tb, ISBN:0198506732 Relationships: is a type of tissue morphogenesis [GO:0048729]; is part of GO:0060429